{
  "term_label": "Unknown molecular function",
  "gene": "UniProtKB:P0DKV0",
  "gene_name": "Putative spermatogenesis-associated protein 31C1",
  "gene_symbol": "SPATA31C1",
  "term_id": "UNKNOWN:0001"
}